nuclear membrane organization [GO:0071763] (biological process) Relationships: is a type of membrane organization [GO:0061024]; is part of nuclear envelope organization [GO:0006998] Definition: A process that is carried out at the cellular level which results in the assembly, arrangement of constituent parts, or disassembly of the nuclear inner or outer membrane. Subtypes: nuclear membrane fusion [GO:0000740], nuclear fragmentation involved in apoptotic nuclear change [GO:0030264], nuclear membrane reassembly [GO:0031468], GO:0051081, nuclear outer membrane organization [GO:0071764], nuclear inner membrane organization [GO:0071765], mitotic nuclear membrane organization [GO:0101024] Sources: GOC:mah Also known as: nuclear membrane organisation, nuclear membrane organization and biogenesis